{
  "gene_name": "Tensin-1",
  "gene": "UniProtKB:Q9HBL0",
  "term_label": "Unknown molecular function",
  "term_id": "UNKNOWN:0001",
  "gene_symbol": "TNS1"
}